{
  "gene_symbol": "AGK",
  "term_id": "GO:0046512",
  "gene_name": "Acylglycerol kinase, mitochondrial",
  "term_label": "sphingosine biosynthetic process",
  "gene": "UniProtKB:Q53H12"
}